{
  "gene": "UniProtKB:Q9UQ10",
  "term_label": "Unknown cellular component",
  "gene_symbol": "DHDH",
  "term_id": "UNKNOWN:0003",
  "gene_name": "Trans-1,2-dihydrobenzene-1,2-diol dehydrogenase"
}